{
  "gene_symbol": "SHPK",
  "term_id": "GO:0050277",
  "gene": "UniProtKB:Q9UHJ6",
  "gene_name": "Sedoheptulokinase",
  "term_label": "sedoheptulokinase activity"
}